{
  "term_label": "fructose transmembrane transport",
  "gene": "UniProtKB:P22732",
  "gene_symbol": "SLC2A5",
  "gene_name": "Solute carrier family 2, facilitated glucose transporter member 5",
  "term_id": "GO:0015755"
}